regulation of translation, ncRNA-mediated [GO:0045974] (biological process) Definition: Any process, mediated by small non-coding RNAs, that modulates the frequency, rate or extent that mRNAs are effectively translated into protein. Sources: GOC:dph, GOC:go_curators, GOC:tb Relationships: is a type of regulation of translation [GO:0006417] Subtypes: positive regulation of translation, ncRNA-mediated [GO:0045975]